{
  "gene_symbol": "TRAPPC3L",
  "gene_name": "Trafficking protein particle complex subunit 3-like protein",
  "term_label": "intra-Golgi vesicle-mediated transport",
  "gene": "UniProtKB:Q5T215",
  "term_id": "GO:0006891"
}